{
  "gene_name": "HLA class II histocompatibility antigen, DR beta 4 chain",
  "gene": "UniProtKB:P13762",
  "gene_symbol": "HLA-DRB4",
  "term_id": "GO:0042605",
  "term_label": "peptide antigen binding"
}